regulation of plasma membrane raft polarization [GO:1903906] (biological process) References: PMID:23575248 Sources: GOC:TermGenie, GOC:als, GO_REF:0000058 Definition: Any process that modulates the frequency, rate or extent of plasma membrane raft polarization. Relationships: is a type of regulation of cellular localization [GO:0060341]; is a type of regulation of plasma membrane organization [GO:1903729]; regulates GO:0044858 Subtypes: negative regulation of plasma membrane raft polarization [GO:1903907], positive regulation of plasma membrane raft polarization [GO:1903908]